molecular_function [GO:0003674] (molecular function) Note: Note that, in addition to forming the root of the molecular function ontology, this term is recommended for the annotation of gene products whose molecular function is unknown. When this term is used for annotation, it indicates that no information was available about the molecular function of the gene product annotated as of the date the annotation was made; the evidence code 'no data' (ND), is used to indicate this. Despite its name, this is not a type of 'function' in the sense typically defined by upper ontologies such as Basic Formal Ontology (BFO). It is instead a BFO:process carried out by a single gene product or complex. Also known as: molecular function Subtypes: cytoskeletal motor activity [GO:0003774], GO:0003824, structural molecule activity [GO:0005198], GO:0005215, binding [GO:0005488], electron transfer activity [GO:0009055], antioxidant activity [GO:0016209], cargo receptor activity [GO:0038024], protein folding chaperone [GO:0044183], translation regulator activity [GO:0045182], nutrient reservoir activity [GO:0045735], molecular transducer activity [GO:0060089], molecular adaptor activity [GO:0060090], toxin activity [GO:0090729], GO:0098772, dirigent protein activity [GO:0102910], molecular carrier activity [GO:0140104], GO:0140110, general transcription initiation factor activity [GO:0140223], GO:0140313, molecular template activity [GO:0140489], fusogenic activity [GO:0140522], GO:0140657, RNA folding chaperone [GO:0140691], GO:0140776, GO:0140777, pore-forming activity [GO:0140911], GO:0140912, GO:0141047, membrane bending activity [GO:0180020], GO:0180024, translation factor activity [GO:0180051] Definition: A molecular process that can be carried out by the action of a single macromolecular machine, usually via direct physical interactions with other molecular entities. Function in this sense denotes an action, or activity, that a gene product (or a complex) performs. Sources: GOC:pdt Regulation: RO_0002212 by negative regulation of molecular function [GO:0044092]; positively regulated by positive regulation of molecular function [GO:0044093]; negatively regulated by modulation by host of viral molecular function [GO:0044868]; regulated by regulation of molecular function [GO:0065009]